{
  "gene": "UniProtKB:Q13061",
  "term_label": "regulation of release of sequestered calcium ion into cytosol by sarcoplasmic reticulum",
  "gene_name": "Triadin",
  "gene_symbol": "TRDN",
  "term_id": "GO:0010880"
}